{
  "gene_symbol": "SFTPA2",
  "gene_name": "Pulmonary surfactant-associated protein A2",
  "term_id": "UNKNOWN:0002",
  "term_label": "Unknown biological process",
  "gene": "UniProtKB:Q8IWL1"
}